{
  "gene_symbol": "SUSD2",
  "gene_name": "Sushi domain-containing protein 2",
  "term_label": "Unknown molecular function",
  "gene": "UniProtKB:Q9UGT4",
  "term_id": "UNKNOWN:0001"
}